{
  "gene": "UniProtKB:P08238",
  "gene_name": "Heat shock protein HSP 90-beta",
  "term_label": "ATP binding",
  "term_id": "GO:0005524",
  "gene_symbol": "HSP90AB1"
}